{
  "gene_name": "Keratin, type II cytoskeletal 73",
  "term_id": "GO:0045109",
  "gene_symbol": "KRT73",
  "gene": "UniProtKB:Q86Y46",
  "term_label": "intermediate filament organization"
}